{
  "term_id": "GO:0005829",
  "term_label": "cytosol",
  "gene_name": "Kelch-like protein 3",
  "gene_symbol": "KLHL3",
  "gene": "UniProtKB:Q9UH77"
}